arylacetonitrilase activity [GO:0047428] (molecular function) Definition: Catalysis of the reaction: 2 H2O + 4-chlorophenylacetonitrile = 4-chlorophenylacetate + NH3. Sources: EC:3.5.5.5 Also known as: arylacetonitrile aminohydrolase activity Relationships: is a type of nitrilase activity [GO:0000257]